{
  "term_label": "neuropeptide receptor activity",
  "gene_symbol": "NPY6R",
  "gene_name": "Putative neuropeptide Y receptor type 6",
  "gene": "UniProtKB:Q99463",
  "term_id": "GO:0008188"
}